{
  "term_id": "GO:0004623",
  "gene_name": "Group XIIA secretory phospholipase A2",
  "term_label": "phospholipase A2 activity",
  "gene": "UniProtKB:Q9BZM1",
  "gene_symbol": "PLA2G12A"
}